{
  "gene_symbol": "EIF2AK3",
  "gene_name": "Eukaryotic translation initiation factor 2-alpha kinase 3",
  "gene": "UniProtKB:Q9NZJ5",
  "term_label": "nucleus",
  "term_id": "GO:0005634"
}